{
  "term_label": "negative regulation of hippo signaling",
  "term_id": "GO:0035331",
  "gene": "UniProtKB:Q9NRL3",
  "gene_name": "Striatin-4",
  "gene_symbol": "STRN4"
}